aromatic-L-amino-acid decarboxylase activity [GO:0004058] (molecular function) Sources: EC:4.1.1.28 Definition: Catalysis of the reaction: L-amino acid + H+ = R-H + CO2. Subtypes: 5-hydroxy-L-tryptophan decarboxylase activity [GO:0036467], GO:0036468, L-tryptophan decarboxylase activity [GO:0036469] Relationships: is a type of carboxy-lyase activity [GO:0016831] Also known as: 5-hydroxytryptophan decarboxylase activity, DOPA decarboxylase activity, L-DOPA decarboxylase activity, aromatic-L-amino-acid carboxy-lyase (tryptamine-forming), hydroxytryptophan decarboxylase activity, tryptophan decarboxylase activity, aromatic amino acid decarboxylase activity, aromatic-L-amino-acid carboxy-lyase activity